negative regulation of iodide transmembrane transport [GO:1904213] (biological process) References: PMID:20392814 Sources: GOC:TermGenie, GO_REF:0000058 Also known as: down regulation of iodide transmembrane transport, down-regulation of iodide transmembrane transport, downregulation of iodide transmembrane transport, inhibition of iodide transmembrane transport Definition: Any process that stops, prevents or reduces the frequency, rate or extent of iodide transmembrane transport. Relationships: is a type of negative regulation of anion transmembrane transport [GO:1903960]; is a type of GO:1904202; is a type of regulation of iodide transmembrane transport [GO:1904212]; negatively regulates GO:1904200